{
  "gene_name": "Pyruvate dehydrogenase protein X component, mitochondrial",
  "term_label": "Unknown biological process",
  "gene_symbol": "PDHX",
  "term_id": "UNKNOWN:0002",
  "gene": "UniProtKB:O00330"
}